{
  "gene_name": "Protein Aster-C",
  "gene_symbol": "GRAMD1C",
  "term_label": "cholesterol binding",
  "term_id": "GO:0015485",
  "gene": "UniProtKB:Q8IYS0"
}